{
  "gene_name": "Sulfotransferase 1A4",
  "term_label": "aryl sulfotransferase activity",
  "gene_symbol": "SULT1A4",
  "gene": "UniProtKB:P0DMN0",
  "term_id": "GO:0004062"
}